{
  "term_id": "GO:0005249",
  "gene": "UniProtKB:Q2I0M4",
  "gene_name": "Leucine-rich repeat-containing protein 26",
  "term_label": "voltage-gated potassium channel activity",
  "gene_symbol": "LRRC26"
}